{
  "term_label": "Unknown cellular component",
  "gene_name": "Oncostatin-M",
  "gene": "UniProtKB:P13725",
  "term_id": "UNKNOWN:0003",
  "gene_symbol": "OSM"
}